{
  "term_label": "plasma membrane",
  "gene": "UniProtKB:P08908",
  "gene_name": "5-hydroxytryptamine receptor 1A",
  "gene_symbol": "HTR1A",
  "term_id": "GO:0005886"
}